{
  "gene_symbol": "WDR91",
  "gene": "UniProtKB:A4D1P6",
  "term_label": "phosphatidylinositol 3-kinase regulator activity",
  "term_id": "GO:0035014",
  "gene_name": "WD repeat-containing protein 91"
}